{
  "gene_symbol": "NASP",
  "term_label": "DNA replication-dependent chromatin assembly",
  "gene_name": "Nuclear autoantigenic sperm protein",
  "gene": "UniProtKB:P49321",
  "term_id": "GO:0006335"
}